{
  "term_id": "GO:0045048",
  "gene": "UniProtKB:Q7L5D6",
  "gene_symbol": "GET4",
  "term_label": "protein insertion into ER membrane",
  "gene_name": "Golgi to ER traffic protein 4 homolog"
}